{
  "gene_name": "Dual specificity tyrosine-phosphorylation-regulated kinase 1A",
  "term_label": "positive regulation of RNA splicing",
  "gene_symbol": "DYRK1A",
  "gene": "UniProtKB:Q13627",
  "term_id": "GO:0033120"
}